{
  "gene_symbol": "CCNP",
  "gene": "UniProtKB:Q9H8S5",
  "gene_name": "Cyclin-P",
  "term_label": "cyclin-dependent protein serine/threonine kinase regulator activity",
  "term_id": "GO:0016538"
}